{
  "gene_symbol": "KANTR",
  "gene": "UniProtKB:A0A1W2PQU2",
  "term_id": "UNKNOWN:0003",
  "gene_name": "KANTR integral membrane protein",
  "term_label": "Unknown cellular component"
}